{
  "term_id": "GO:0007165",
  "term_label": "signal transduction",
  "gene": "UniProtKB:Q8NG98",
  "gene_symbol": "OR7D4",
  "gene_name": "Olfactory receptor 7D4"
}